{
  "gene": "UniProtKB:O15264",
  "gene_symbol": "MAPK13",
  "term_id": "GO:0005634",
  "gene_name": "Mitogen-activated protein kinase 13",
  "term_label": "nucleus"
}